{
  "gene_symbol": "POLR1A",
  "term_id": "GO:0042790",
  "term_label": "nucleolar large rRNA transcription by RNA polymerase I",
  "gene_name": "DNA-directed RNA polymerase I subunit RPA1",
  "gene": "UniProtKB:O95602"
}